positive regulation of protein localization to phagocytic vesicle [GO:1905171] (BP) Definition: Any process that activates or increases the frequency, rate or extent of protein localization to phagocytic vesicle. Also known as: positive regulation of protein localisation in phagocytic vesicle, positive regulation of protein localisation to phagocytic vesicle, positive regulation of protein localisation to phagosome, positive regulation of protein localization in phagocytic vesicle, positive regulation of protein recruitment to phagosome, up regulation of protein localisation in phagocytic vesicle, up regulation of protein localisation to phagocytic vesicle, up regulation of protein localisation to phagosome, up regulation of protein localization in phagocytic vesicle, up regulation of protein localization to phagocytic vesicle, up regulation of protein recruitment to phagosome, up-regulation of protein localisation in phagocytic vesicle, up-regulation of protein localisation to phagocytic vesicle, up-regulation of protein localisation to phagosome, up-regulation of protein localization in phagocytic vesicle, up-regulation of protein localization to phagocytic vesicle, up-regulation of protein recruitment to phagosome, upregulation of protein localisation in phagocytic vesicle, upregulation of protein localisation to phagocytic vesicle, upregulation of protein localisation to phagosome, upregulation of protein localization in phagocytic vesicle, upregulation of protein localization to phagocytic vesicle, upregulation of protein recruitment to phagosome, activation of protein localisation in phagocytic vesicle, activation of protein localisation to phagocytic vesicle, activation of protein localisation to phagosome, activation of protein localization in phagocytic vesicle, activation of protein localization to phagocytic vesicle, activation of protein recruitment to phagosome References: PMID:23303671 Sources: GOC:PARL, GOC:TermGenie, GOC:bf, GO_REF:0000058 Relationships: is a type of positive regulation of protein localization [GO:1903829]; is a type of regulation of protein localization to phagocytic vesicle [GO:1905169]; positively regulates protein localization to phagocytic vesicle [GO:1905161]